{
  "term_label": "positive regulation of T cell mediated cytotoxicity",
  "gene": "UniProtKB:P01893",
  "gene_name": "Putative HLA class I histocompatibility antigen, alpha chain H",
  "term_id": "GO:0001916",
  "gene_symbol": "HLA-H"
}